{
  "term_label": "protein kinase activator activity",
  "gene_name": "Retinoic acid-induced protein 3",
  "gene": "UniProtKB:Q8NFJ5",
  "term_id": "GO:0030295",
  "gene_symbol": "GPRC5A"
}